{
  "term_id": "GO:0006383",
  "term_label": "transcription by RNA polymerase III",
  "gene": "UniProtKB:Q9Y5Q9",
  "gene_symbol": "GTF3C3",
  "gene_name": "General transcription factor 3C polypeptide 3"
}